{
  "gene_name": "IQCJ-SCHIP1 readthrough transcript protein",
  "term_label": "plasma membrane",
  "gene": "UniProtKB:B3KU38",
  "gene_symbol": "IQCJ-SCHIP1",
  "term_id": "GO:0005886"
}